{
  "term_label": "cytokine activity",
  "gene": "UniProtKB:P13232",
  "term_id": "GO:0005125",
  "gene_name": "Interleukin-7",
  "gene_symbol": "IL7"
}